{
  "gene_symbol": "OR2F2",
  "gene": "UniProtKB:O95006",
  "term_label": "plasma membrane",
  "gene_name": "Olfactory receptor 2F2",
  "term_id": "GO:0005886"
}